{
  "term_id": "GO:0005829",
  "gene_symbol": "NLRC5",
  "gene": "UniProtKB:Q86WI3",
  "gene_name": "Protein NLRC5",
  "term_label": "cytosol"
}